pollen tube adhesion [GO:0009865] (biological process) Definition: The process in which the pollen tube adheres to cells of the stigma and style. References: PMID:12602877 Sources: GOC:tair_curators Relationships: is a type of biological process involved in intraspecies interaction between organisms [GO:0051703]; is a type of GO:0098609; is part of GO:0009875; is part of GO:0048868